{
  "gene_symbol": "CTSD",
  "term_id": "GO:0004190",
  "gene_name": "Cathepsin D",
  "term_label": "aspartic-type endopeptidase activity",
  "gene": "UniProtKB:P07339"
}